{
  "gene_symbol": "SLC35G2",
  "term_label": "Unknown molecular function",
  "gene": "UniProtKB:Q8TBE7",
  "gene_name": "Solute carrier family 35 member G2",
  "term_id": "UNKNOWN:0001"
}